RAD6-UBR2 ubiquitin ligase complex [GO:1990305] (cellular component) Definition: A ubiquitin ligase complex consisting of RAD6 and UBR2 components. It may act in a quality control pathway for proteins synthesized on cytosolic ribosomes. The UBR2 component lacks sequence motifs required for N-end rule degradation. Also known as: RAD6-UBR2 complex References: PMID:15504724 Sources: GOC:bhm Relationships: is a type of intracellular protein-containing complex [GO:0140535]; is a type of GO:1990234 Note: This complex has been identified in Saccharomyces cerevisiae (P19812) - see PMID:15504724